negative regulation of behavioral fear response [GO:2000986] (biological process) Definition: Any process that stops, prevents or reduces the frequency, rate or extent of behavioral fear response. Sources: GOC:obol Also known as: negative regulation of behavioural fear response Relationships: is a type of negative regulation of defense response [GO:0031348]; is a type of negative regulation of behavior [GO:0048521]; is a type of GO:1903366; is a type of regulation of behavioral fear response [GO:2000822]; negatively regulates behavioral fear response [GO:0001662]